{
  "term_id": "GO:0004198",
  "gene_symbol": "CAPN11",
  "gene_name": "Calpain-11",
  "term_label": "calcium-dependent cysteine-type endopeptidase activity",
  "gene": "UniProtKB:Q9UMQ6"
}